{
  "gene_name": "Nuclear receptor coactivator 7",
  "term_label": "transcription coactivator activity",
  "term_id": "GO:0003713",
  "gene": "UniProtKB:Q8NI08",
  "gene_symbol": "NCOA7"
}